syn-pimaradiene 6beta-hydroxylase activity [GO:0102612] (molecular function) Relationships: is_a GO:0016709 References: PMID:22215681 Sources: GOC:pz Definition: Catalysis of the reaction: 9beta-pimara-7,15-diene + NADPH + O2 + H+ = 6beta-hydroxy-syn-pimaradiene + NADP + H2O.